{
  "term_id": "GO:0042391",
  "gene_name": "Potassium voltage-gated channel subfamily H member 4",
  "term_label": "regulation of membrane potential",
  "gene": "UniProtKB:Q9UQ05",
  "gene_symbol": "KCNH4"
}